{
  "gene": "UniProtKB:P63241",
  "term_id": "GO:0003746",
  "term_label": "translation elongation factor activity",
  "gene_name": "Eukaryotic translation initiation factor 5A-1",
  "gene_symbol": "EIF5A"
}